tryparedoxin peroxidase activity [GO:0033196] (molecular function) Relationships: is a type of peroxidase activity [GO:0004601] Also known as: TXNPx activity References: PMID:32388269 Sources: GOC:mah Definition: Catalysis of the reaction: tryparedoxin + hydrogen peroxide = tryparedoxin disulfide + H2O.